{
  "term_label": "keratin filament",
  "gene": "UniProtKB:P05783",
  "term_id": "GO:0045095",
  "gene_symbol": "KRT18",
  "gene_name": "Keratin, type I cytoskeletal 18"
}